{
  "term_id": "GO:0006357",
  "term_label": "regulation of transcription by RNA polymerase II",
  "gene_name": "Max-binding protein MNT",
  "gene": "UniProtKB:Q99583",
  "gene_symbol": "MNT"
}